{
  "term_label": "actin cytoskeleton organization",
  "gene": "UniProtKB:Q96PE2",
  "term_id": "GO:0030036",
  "gene_symbol": "ARHGEF17",
  "gene_name": "Rho guanine nucleotide exchange factor 17"
}